{
  "term_label": "Unknown cellular component",
  "gene_symbol": "A0A1W2PRE2",
  "gene_name": "Uncharacterized protein",
  "term_id": "UNKNOWN:0003",
  "gene": "UniProtKB:A0A1W2PRE2"
}